ciliary body morphogenesis [GO:0061073] (biological process) Sources: GOC:dph Definition: The process in which the ciliary body generated and organized. The ciliary body is the circumferential tissue inside the eye composed of the ciliary muscle and ciliary processes. Relationships: is a type of GO:0009653; BFO_0000050 camera-type eye morphogenesis [GO:0048593]